{
  "gene_symbol": "CD3G",
  "term_id": "GO:0045059",
  "gene_name": "T-cell surface glycoprotein CD3 gamma chain",
  "term_label": "positive thymic T cell selection",
  "gene": "UniProtKB:P09693"
}